{
  "term_id": "GO:0005912",
  "term_label": "adherens junction",
  "gene_symbol": "ADD1",
  "gene_name": "Alpha-adducin",
  "gene": "UniProtKB:P35611"
}